female germ-line cyst formation [GO:0048135] (biological process) Relationships: is a type of germ-line cyst formation [GO:0048134]; is part of GO:0048477 Definition: Formation of a group of interconnected cells derived from a single female gonial founder cell. Subtypes: germarium-derived female germ-line cyst formation [GO:0030727] References: PMID:10370240 Sources: GOC:jid Also known as: female germline cyst formation